epidermal growth factor binding [GO:0048408] (MF) Definition: Binding to epidermal growth factor. Sources: GOC:dgh Relationships: is_a GO:0019838; is a type of GO:0042562 Also known as: EGF binding